{
  "gene": "UniProtKB:Q76NI1",
  "gene_symbol": "KNDC1",
  "term_id": "GO:0032045",
  "gene_name": "Kinase non-catalytic C-lobe domain-containing protein 1",
  "term_label": "guanyl-nucleotide exchange factor complex"
}